{
  "gene_name": "Zinc finger protein 483",
  "gene_symbol": "ZNF483",
  "term_id": "GO:0006357",
  "term_label": "regulation of transcription by RNA polymerase II",
  "gene": "UniProtKB:Q8TF39"
}